{
  "gene_name": "Na(+)_citrate cotransporter",
  "term_label": "succinate transmembrane transporter activity",
  "gene_symbol": "SLC13A5",
  "gene": "UniProtKB:Q86YT5",
  "term_id": "GO:0015141"
}